fucosylgalactoside 3-alpha-galactosyltransferase activity [GO:0004381] (MF) Relationships: is_a GO:0035250 Definition: Catalysis of the reaction: UDP-galactose + glycoprotein-alpha-L-fucosyl-(1,2)-D-galactose = UDP + glycoprotein-alpha-D-galactosyl-(1,3)-(alpha-L-fucosyl-(1,2))-D-galactose. Sources: EC:2.4.1.37 Also known as: glycoprotein-fucosylgalactoside alpha-galactosyltransferase activity, [blood group substance] alpha-galactosyltransferase activity, blood-group substance B-dependent galactosyltransferase activity, blood-group substance beta-dependent galactosyltransferase activity, histo-blood group B transferase activity, histo-blood substance beta-dependent galactosyltransferase activity, B transferase activity, UDP-galactose:alpha-L-fucosyl-(1,2)-D-galactoside 3-alpha-D-galactosyltransferase activity, UDP-galactose:alpha-L-fucosyl-(1->2)-D-galactoside 3-alpha-D-galactosyltransferase activity, UDPgalactose:O-alpha-L-fucosyl(1,2)D-galactose alpha-D-galactosyltransferase activity, UDPgalactose:O-alpha-L-fucosyl(1->2)D-galactose alpha-D-galactosyltransferase activity, UDPgalactose:alpha-L-fucosyl-(1,2)-D-galactoside 3-alpha-D-galactosyltransferase activity, UDPgalactose:alpha-L-fucosyl-(1->2)-D-galactoside 3-alpha-D-galactosyltransferase activity, UDPgalactose:glycoprotein-alpha-L-fucosyl-(1,2)-D-galactose 3-alpha-D-galactosyltransferase activity, fucosylglycoprotein 3-alpha-galactosyltransferase activity, histo-blood substance B-dependent galactosyltransferase activity